{
  "gene_name": "Double C2-like domain-containing protein alpha",
  "term_label": "positive regulation of calcium ion-dependent exocytosis",
  "term_id": "GO:0045956",
  "gene_symbol": "DOC2A",
  "gene": "UniProtKB:Q14183"
}